{
  "gene_symbol": "GADD45G",
  "gene": "UniProtKB:O95257",
  "term_id": "GO:0005737",
  "term_label": "cytoplasm",
  "gene_name": "Growth arrest and DNA damage-inducible protein GADD45 gamma"
}